{
  "gene_symbol": "FCGR3B",
  "term_label": "cell surface receptor signaling pathway",
  "term_id": "GO:0007166",
  "gene": "UniProtKB:O75015",
  "gene_name": "Low affinity immunoglobulin gamma Fc region receptor III-B"
}